cellular response to hexose stimulus [GO:0071331] (biological process) Sources: GOC:mah Definition: Any process that results in a change in state or activity of a cell (in terms of movement, secretion, enzyme production, gene expression, etc.) as a result of a hexose stimulus. Relationships: is a type of response to hexose [GO:0009746]; is a type of cellular response to monosaccharide stimulus [GO:0071326] Subtypes: GO:0071332, GO:0071333, GO:0071334, GO:1905378, GO:1905583